{
  "term_id": "UNKNOWN:0001",
  "gene_name": "UPF0739 protein C1orf74",
  "gene_symbol": "C1orf74",
  "gene": "UniProtKB:Q96LT6",
  "term_label": "Unknown molecular function"
}